{
  "gene_symbol": "SAP30",
  "term_id": "GO:0006355",
  "gene_name": "Histone deacetylase complex subunit SAP30",
  "gene": "UniProtKB:O75446",
  "term_label": "regulation of DNA-templated transcription"
}